{
  "term_id": "GO:0001503",
  "gene_name": "Tetranectin",
  "term_label": "ossification",
  "gene": "UniProtKB:P05452",
  "gene_symbol": "CLEC3B"
}